{
  "gene_symbol": "STAU1",
  "gene": "UniProtKB:O95793",
  "gene_name": "Double-stranded RNA-binding protein Staufen homolog 1",
  "term_label": "intracellular mRNA localization",
  "term_id": "GO:0008298"
}